{
  "term_id": "GO:0005144",
  "gene_symbol": "IL13",
  "term_label": "interleukin-13 receptor binding",
  "gene_name": "Interleukin-13",
  "gene": "UniProtKB:P35225"
}